negative regulation of serotonin uptake [GO:0051612] (biological process) Definition: Any process that stops, prevents, or reduces the frequency, rate or extent of the directed movement of serotonin into a cell. Sources: GOC:ai Also known as: down regulation of serotonin uptake, down-regulation of serotonin uptake, downregulation of serotonin uptake, negative regulation of 5-HT uptake, negative regulation of 5-hydroxytryptamine uptake, negative regulation of 5HT uptake, negative regulation of serotonin import Relationships: is a type of negative regulation of neurotransmitter uptake [GO:0051581]; is a type of regulation of serotonin uptake [GO:0051611]; negatively regulates serotonin uptake [GO:0051610] Subtypes: GO:0051614